{
  "gene_name": "Elongator complex protein 6",
  "gene": "UniProtKB:Q0PNE2",
  "gene_symbol": "ELP6",
  "term_label": "Unknown molecular function",
  "term_id": "UNKNOWN:0001"
}